{
  "gene_name": "Tripartite motif-containing protein 16-like protein",
  "gene_symbol": "TRIM16L",
  "gene": "UniProtKB:Q309B1",
  "term_id": "UNKNOWN:0001",
  "term_label": "Unknown molecular function"
}